{
  "term_id": "GO:0005794",
  "gene": "UniProtKB:Q8N3Y3",
  "term_label": "Golgi apparatus",
  "gene_name": "Xylosyl- and glucuronyltransferase LARGE2",
  "gene_symbol": "LARGE2"
}